{
  "gene": "UniProtKB:Q13485",
  "gene_symbol": "SMAD4",
  "gene_name": "Mothers against decapentaplegic homolog 4",
  "term_label": "RNA polymerase II cis-regulatory region sequence-specific DNA binding",
  "term_id": "GO:0000978"
}